cytoplasmic side of apical plasma membrane [GO:0098592] (CC) Relationships: is a type of GO:0009898; is part of GO:0016324 Sources: GOC:ab, GOC:dos Definition: The side (leaflet) of the apical region of the plasma membrane that faces the cytoplasm.